{
  "gene": "UniProtKB:P36269",
  "term_id": "GO:0006751",
  "term_label": "glutathione catabolic process",
  "gene_symbol": "GGT5",
  "gene_name": "Glutathione hydrolase 5 proenzyme"
}